{
  "gene_name": "Phospholipase DDHD1",
  "gene": "UniProtKB:Q8NEL9",
  "gene_symbol": "DDHD1",
  "term_id": "GO:0005737",
  "term_label": "cytoplasm"
}